cardiac muscle cell contraction [GO:0086003] (biological process) Definition: The actin filament-based process in which cytoplasmic actin filaments slide past one another resulting in contraction of a cardiac muscle cell. Sources: GOC:BHF, GOC:mtg_cardiac_conduct_nov11 Regulation: regulated by GO:0086004; positively regulated by positive regulation of cardiac muscle cell contraction [GO:0106134]; negatively regulated by negative regulation of cardiac muscle cell contraction [GO:0106135] Relationships: is a type of actin-mediated cell contraction [GO:0070252]; is part of cardiac muscle contraction [GO:0060048]